{
  "term_id": "UNKNOWN:0001",
  "gene_name": "Alanine aminotransferase 2",
  "gene_symbol": "GPT2",
  "term_label": "Unknown molecular function",
  "gene": "UniProtKB:Q8TD30"
}